protein-N(PI)-phosphohistidine-galactitol phosphotransferase system transmembrane transporter activity [GO:0022875] (molecular function) Sources: GOC:mtg_transport, ISBN:0815340729 Definition: Catalysis of the PEP-dependent, phosphoryl transfer-driven transport of substances across a membrane. The transport happens by catalysis of the reaction: protein N-phosphohistidine + galactitol(out) = protein histidine + galactitol phosphate(in). This differs from primary and secondary active transport in that the solute is modified during transport. Relationships: is a type of protein-N(PI)-phosphohistidine-sugar phosphotransferase activity [GO:0008982]; is a type of galactitol transmembrane transporter activity [GO:0015577] Also known as: galactitol PTS transporter activity